pyrimidine nucleobase transport [GO:0015855] (biological process) Also known as: pyrimidine base transmembrane transport, pyrimidine base transport, pyrimidine transmembrane transport, pyrimidine transport Subtypes: cytosine transport [GO:0015856], uracil transport [GO:0015857], thymine transport [GO:0035364], pyrimidine nucleobase transmembrane transport [GO:1904082] Relationships: is_a nucleobase transport [GO:0015851] Definition: The directed movement of pyrimidine nucleobases, one of the two classes of nitrogen-containing ring compounds found in DNA and RNA, into, out of or within a cell, or between cells, by means of some agent such as a transporter or pore. Sources: GOC:ai